{
  "term_label": "aspartate biosynthetic process",
  "gene_name": "Aspartate aminotransferase, cytoplasmic",
  "term_id": "GO:0006532",
  "gene_symbol": "GOT1",
  "gene": "UniProtKB:P17174"
}